adult foraging behavior [GO:0060757] (biological process) Sources: GOC:dph, GOC:tb Relationships: is a type of foraging behavior [GO:0060756] Definition: Behavior by which an adult locates food.